{
  "gene_name": "Geminin",
  "gene_symbol": "GMNN",
  "term_label": "transcription coregulator activity",
  "term_id": "GO:0003712",
  "gene": "UniProtKB:O75496"
}